{
  "gene": "UniProtKB:P13688",
  "gene_name": "Carcinoembryonic antigen-related cell adhesion molecule 1",
  "term_id": "GO:0009986",
  "gene_symbol": "CEACAM1",
  "term_label": "cell surface"
}